positive regulation of filamentous growth of a population of unicellular organisms in response to biotic stimulus [GO:1900445] (biological process) Also known as: up regulation of filamentous growth of a population of unicellular organisms in response to biotic stimulus, up-regulation of filamentous growth of a population of unicellular organisms in response to biotic stimulus, upregulation of filamentous growth of a population of unicellular organisms in response to biotic stimulus, activation of filamentous growth of a population of unicellular organisms in response to biotic stimulus Sources: GOC:TermGenie, GOC:di Relationships: is a type of positive regulation of response to biotic stimulus [GO:0002833]; is a type of GO:1900430; is a type of GO:1900443; positively regulates filamentous growth of a population of unicellular organisms in response to biotic stimulus [GO:0036180] Definition: Any process that activates or increases the frequency, rate or extent of filamentous growth of a population of unicellular organisms in response to biotic stimulus.